{
  "gene": "UniProtKB:O60508",
  "gene_name": "Pre-mRNA-processing factor 17",
  "gene_symbol": "CDC40",
  "term_id": "GO:0000398",
  "term_label": "mRNA splicing, via spliceosome"
}